{
  "gene_name": "Microtubule-associated proteins 1A_1B light chain 3B",
  "gene": "UniProtKB:Q9GZQ8",
  "gene_symbol": "MAP1LC3B",
  "term_id": "GO:0000423",
  "term_label": "mitophagy"
}